negative regulation of CD8-positive, alpha-beta T cell extravasation [GO:2000450] (biological process) Sources: GOC:obol Definition: Any process that stops, prevents or reduces the frequency, rate or extent of CD8-positive, alpha-beta T cell extravasation. Subtypes: negative regulation of CD8-positive, alpha-beta cytotoxic T cell extravasation [GO:2000453], GO:2000456 Relationships: is a type of GO:2000408; is a type of regulation of CD8-positive, alpha-beta T cell extravasation [GO:2000449]; negatively regulates GO:0035697